{
  "gene_name": "RNA binding protein fox-1 homolog 2",
  "gene_symbol": "RBFOX2",
  "term_label": "regulation of alternative mRNA splicing, via spliceosome",
  "gene": "UniProtKB:O43251",
  "term_id": "GO:0000381"
}